{
  "term_label": "Unknown biological process",
  "term_id": "UNKNOWN:0002",
  "gene_symbol": "FAM216A",
  "gene_name": "Protein FAM216A",
  "gene": "UniProtKB:Q8WUB2"
}